anterior cibarial plate development [GO:0048722] (biological process) Sources: GOC:rc Relationships: is a type of anatomical structure development [GO:0048856]; is part of clypeo-labral disc development [GO:0035213] Definition: The process whose specific outcome is the progression of the anterior cibarial plate over time, from their formation to the mature structure.